{
  "gene_name": "Protein FAM174C",
  "gene": "UniProtKB:Q9BVV8",
  "gene_symbol": "FAM174C",
  "term_label": "Unknown biological process",
  "term_id": "UNKNOWN:0002"
}